{
  "term_label": "ubiquitin conjugating enzyme binding",
  "term_id": "GO:0031624",
  "gene_symbol": "RNF217",
  "gene": "UniProtKB:Q8TC41",
  "gene_name": "E3 ubiquitin-protein ligase RNF217"
}